intracellular ammonium homeostasis [GO:0097275] (biological process) References: PMID:12695560 Sources: GOC:yaf Relationships: is a type of intracellular chemical homeostasis [GO:0055082]; is a type of ammonium homeostasis [GO:0097272] Definition: A homeostatic process involved in the maintenance of a steady state level of ammonium within a cell. Also known as: cellular ammonia homeostasis, cellular ammonium homeostasis